leukotriene B4 receptor activity [GO:0001632] (molecular function) Sources: GOC:ai, ISBN:0198506732 Also known as: BLT receptor Definition: Combining with leukotriene B4, LTB4, to initiate a change in cell activity. Leukotriene B4 is also known as (6Z, 8E, 10E, 14Z)-(5S, 12R)-5,12-dihydroxyicosa-6,8,10,14-tetraen-1-oate. Relationships: is a type of leukotriene receptor activity [GO:0004974]